{
  "gene_symbol": "TOP2A",
  "gene": "UniProtKB:P11388",
  "term_label": "resolution of meiotic recombination intermediates",
  "term_id": "GO:0000712",
  "gene_name": "DNA topoisomerase 2-alpha"
}